{
  "gene": "UniProtKB:Q9Y6H6",
  "term_label": "regulation of heart rate by cardiac conduction",
  "term_id": "GO:0086091",
  "gene_name": "Potassium voltage-gated channel subfamily E member 3",
  "gene_symbol": "KCNE3"
}